{
  "gene_name": "Mitochondrial inner membrane protein OXA1L",
  "gene": "UniProtKB:Q15070",
  "term_label": "membrane insertase activity",
  "gene_symbol": "OXA1L",
  "term_id": "GO:0032977"
}